{
  "gene_name": "Rho-related GTP-binding protein RhoE",
  "gene": "UniProtKB:P61587",
  "term_id": "GO:0007015",
  "gene_symbol": "RND3",
  "term_label": "actin filament organization"
}